{
  "gene_symbol": "LINC02881",
  "gene_name": "Uncharacterized protein encoded by LINC02881",
  "gene": "UniProtKB:B7Z368",
  "term_label": "Unknown cellular component",
  "term_id": "UNKNOWN:0003"
}